AMPA glutamate receptor activity [GO:0004971] (molecular function) References: PMID:10049997, PMID:8804111 Sources: GOC:mah Note: Note that this term represents an activity and not a gene product. Consider also annotating to the molecular function terms 'ionotropic glutamate receptor activity ; GO:0004970' and 'cation channel activity ; GO:0005261'. Definition: An ionotropic glutamate receptor activity that exhibits fast gating by glutamate and acts by opening a cation channel permeable to sodium, potassium, and, in the absence of a GluR2 subunit, calcium. Also known as: AMPA receptor activity, alpha-amino-3-hydroxy-5-methyl-4-isoxazole propionate selective glutamate receptor activity Regulation: regulated by regulation of AMPA receptor activity [GO:2000311]; positively regulated by GO:2000969 Relationships: is a type of glutamate-gated receptor activity [GO:0004970]